{
  "term_id": "GO:0005248",
  "term_label": "voltage-gated sodium channel activity",
  "gene": "UniProtKB:Q9UQD0",
  "gene_symbol": "SCN8A",
  "gene_name": "Sodium channel protein type 8 subunit alpha"
}